response to purvalanol A [GO:1901560] (biological process) Subtypes: cellular response to purvalanol A [GO:0072754] Sources: GOC:TermGenie Relationships: is a type of GO:0014074 Definition: Any process that results in a change in state or activity of a cell or an organism (in terms of movement, secretion, enzyme production, gene expression, etc.) as a result of a purvalanol A stimulus.